{
  "gene": "UniProtKB:Q9NPH5",
  "gene_symbol": "NOX4",
  "term_label": "NADPH oxidase complex",
  "term_id": "GO:0043020",
  "gene_name": "NADPH oxidase 4"
}